{
  "gene_symbol": "SHISA5",
  "term_id": "GO:0005783",
  "gene_name": "Protein shisa-5",
  "term_label": "endoplasmic reticulum",
  "gene": "UniProtKB:Q8N114"
}